{
  "term_label": "Unknown cellular component",
  "gene": "UniProtKB:Q96CN4",
  "gene_symbol": "EVI5L",
  "gene_name": "EVI5-like protein",
  "term_id": "UNKNOWN:0003"
}